positive regulation of synapse assembly [GO:0051965] (BP) Relationships: is a type of positive regulation of nervous system development [GO:0051962]; is a type of regulation of synapse assembly [GO:0051963]; is a type of GO:1901890; positively regulates synapse assembly [GO:0007416] Definition: Any process that activates, maintains or increases the frequency, rate or extent of synapse assembly, the aggregation, arrangement and bonding together of a set of components to form a synapse. Also known as: positive regulation of synapse biogenesis, positive regulation of synaptogenesis, up regulation of synapse assembly, up-regulation of synapse assembly, upregulation of synapse assembly, activation of synapse assembly, stimulation of synapse assembly Sources: GOC:ai, GOC:pr Subtypes: positive regulation of synaptic assembly at neuromuscular junction [GO:0045887], positive regulation of excitatory synapse assembly [GO:1904891], positive regulation of inhibitory synapse assembly [GO:1905704]